response to insecticide [GO:0017085] (biological process) Definition: Any process that results in a change in state or activity of a cell or an organism (in terms of movement, secretion, enzyme production, gene expression, etc.) as a result of an insecticide stimulus. Insecticides are chemicals used to kill insects. Sources: GOC:curators Also known as: insecticide resistance, insecticide susceptibility/resistance Relationships: is a type of response to toxic substance [GO:0009636] Subtypes: response to DDT [GO:0046680], response to carbamate [GO:0046681], response to cyclodiene [GO:0046682], response to pyrethroid [GO:0046684]